ferredoxin metabolic process [GO:0006124] (biological process) Sources: ISBN:0198506732 Also known as: ferredoxin metabolism Definition: The chemical reactions and pathways involving ferredoxin, any simple, nonenzymatic iron-sulfur protein that is characterized by having equal numbers of atoms of iron and labile sulfur. Iron and sulfur atoms are present in one or two clusters of two or four atoms of each. Relationships: is a type of GO:0019538